aldehyde catabolic process [GO:0046185] (biological process) Definition: The chemical reactions and pathways resulting in the breakdown of aldehydes, any organic compound with the formula R-CH=O. Sources: GOC:ai Also known as: aldehyde breakdown, aldehyde catabolism, aldehyde degradation Relationships: is_a aldehyde metabolic process [GO:0006081]; is a type of GO:0009056 Subtypes: GO:0009436, glyceraldehyde-3-phosphate catabolic process [GO:0019683], aldosterone catabolic process [GO:0032343], pyridoxal phosphate catabolic process [GO:0032361], vanillin catabolic process [GO:0042190], acetaldehyde catabolic process [GO:0046187], formaldehyde catabolic process [GO:0046294], methylglyoxal catabolic process [GO:0051596], glyoxal catabolic process [GO:1903190]